{
  "gene_symbol": "TMEM126B",
  "term_label": "Unknown molecular function",
  "term_id": "UNKNOWN:0001",
  "gene_name": "Complex I assembly factor TMEM126B, mitochondrial",
  "gene": "UniProtKB:Q8IUX1"
}